{
  "gene": "UniProtKB:P02708",
  "gene_name": "Acetylcholine receptor subunit alpha",
  "term_label": "acetylcholine receptor signaling pathway",
  "term_id": "GO:0095500",
  "gene_symbol": "CHRNA1"
}